{
  "gene_name": "E3 ubiquitin-protein ligase TRIM38",
  "gene": "UniProtKB:O00635",
  "gene_symbol": "TRIM38",
  "term_id": "GO:0010468",
  "term_label": "regulation of gene expression"
}